{
  "gene_name": "GTPase IMAP family member 7",
  "gene_symbol": "GIMAP7",
  "term_label": "Unknown biological process",
  "term_id": "UNKNOWN:0002",
  "gene": "UniProtKB:Q8NHV1"
}